{
  "gene_name": "Solute carrier organic anion transporter family member 1C1",
  "term_label": "basolateral plasma membrane",
  "gene_symbol": "SLCO1C1",
  "term_id": "GO:0016323",
  "gene": "UniProtKB:Q9NYB5"
}